{
  "gene_symbol": "BEX1",
  "term_label": "signal transduction",
  "term_id": "GO:0007165",
  "gene_name": "Protein BEX1",
  "gene": "UniProtKB:Q9HBH7"
}